cAMP-dependent protein kinase inhibitor activity [GO:0004862] (molecular function) Sources: GOC:mah Definition: Binds to and stops, prevents or reduces the activity of a cAMP-dependent protein kinase. Relationships: is a type of cAMP-dependent protein kinase regulator activity [GO:0008603]; is_a protein serine/threonine kinase inhibitor activity [GO:0030291]; negatively regulates GO:0004691